regulation of keratinocyte migration [GO:0051547] (biological process) Definition: Any process that modulates the frequency, rate or extent of keratinocyte migration. Sources: GOC:ai Subtypes: negative regulation of keratinocyte migration [GO:0051548], GO:0051549 Relationships: is a type of regulation of epithelial cell migration [GO:0010632]; regulates keratinocyte migration [GO:0051546]